myoblast fate determination [GO:0007518] (biological process) Relationships: is a type of cell fate determination [GO:0001709]; is part of myoblast fate commitment [GO:0048625] Subtypes: myoblast fate determination involved in skeletal muscle regeneration [GO:0014837] Sources: CL:0000056, GOC:go_curators Definition: The cell fate determination process in which a cell becomes capable of differentiating autonomously into a myoblast regardless of its environment; upon determination, the cell fate cannot be reversed. A myoblast is a mononucleate cell type that, by fusion with other myoblasts, gives rise to the myotubes that eventually develop into skeletal muscle fibers.